{
  "term_id": "GO:0055085",
  "gene": "UniProtKB:Q8NBS3",
  "term_label": "transmembrane transport",
  "gene_name": "Solute carrier family 4 member 11",
  "gene_symbol": "SLC4A11"
}